promoter-terminator loop anchoring activity [GO:0140586] (MF) Definition: Bridging together a cis-regulatory element and a terminator DNA sequences on the chromatin, holding two loop anchors together, maintaining a chromatin loop. Note: Note that GO does not separately defines enhancers, since this concept is very close to that of cis-regulatory elements. However the literature refers to 'promoter-enhancer loops' to describe loops that bring together cis-regulatory elements. Note also that while SO defines 'promoter' as the core promoter, here it is used to mean a cis-regulatory element. References: PMID:19933151 Also known as: terminator-promoter loop anchoring activity Relationships: is a type of chromatin loop anchoring activity [GO:0140587]